{
  "term_label": "base-excision repair, AP site formation",
  "gene_name": "N-glycosylase_DNA lyase",
  "gene": "UniProtKB:O15527",
  "gene_symbol": "OGG1",
  "term_id": "GO:0006285"
}